double-strand break repair via transcription-associated homologous recombination [GO:0106400] (biological process) Definition: A mechanism of homologous recombination and DNA repair in which transcript RNA is used as a template for DSB repair. Relationships: is a type of double-strand break repair via homologous recombination [GO:0000724] References: PMID:25186730